positive regulation of antigen processing and presentation of peptide antigen [GO:0002585] (biological process) Sources: GOC:add Definition: Any process that activates or increases the frequency, rate, or extent of antigen processing and presentation of peptide antigen. Also known as: positive regulation of peptide antigen processing and presentation, up regulation of antigen processing and presentation of peptide antigen, up-regulation of antigen processing and presentation of peptide antigen, upregulation of antigen processing and presentation of peptide antigen, activation of antigen processing and presentation of peptide antigen, stimulation of antigen processing and presentation of peptide antigen Subtypes: positive regulation of antigen processing and presentation of peptide antigen via MHC class II [GO:0002588], positive regulation of antigen processing and presentation of peptide antigen via MHC class I [GO:0002591], GO:0002597, positive regulation of proteolysis associated with antigen processing and presentation [GO:0002630], GO:1901041 Relationships: is a type of positive regulation of antigen processing and presentation [GO:0002579]; is a type of regulation of antigen processing and presentation of peptide antigen [GO:0002583]; positively regulates GO:0048002